starch metabolic process [GO:0005982] (biological process) Relationships: is_a glucan metabolic process [GO:0044042] Also known as: starch metabolism Regulation: regulated by GO:2000904 Definition: The chemical reactions and pathways involving starch, the most important reserve polysaccharide in plants. It is a glucan consisting of two components, amylose and amylopectin, which are both glucose homopolymers. Starch is synthesized as a temporary storage form of carbon and can be catabolized to produce sucrose. Sources: ISBN:0198506732 Subtypes: GO:0005983, GO:0019252